{
  "term_label": "Unknown biological process",
  "gene_name": "PDZ domain-containing protein GIPC2",
  "gene": "UniProtKB:Q8TF65",
  "term_id": "UNKNOWN:0002",
  "gene_symbol": "GIPC2"
}